{
  "gene_symbol": "ANAPC11",
  "gene": "UniProtKB:Q9NYG5",
  "term_id": "GO:0016567",
  "gene_name": "Anaphase-promoting complex subunit 11",
  "term_label": "protein ubiquitination"
}